sulfate import across plasma membrane [GO:1902434] (biological process) Definition: The directed movement of sulfate from outside of a cell, across the plasma membrane and into the cytosol. References: PMID:14723223 Sources: GOC:TermGenie Also known as: sulfate import into cell, sulphate import into cell Relationships: is a type of GO:0098658; is a type of sulfate transmembrane transport [GO:1902358]